{
  "term_label": "nucleolus",
  "gene_symbol": "RIOX2",
  "gene": "UniProtKB:Q8IUF8",
  "gene_name": "Ribosomal oxygenase 2",
  "term_id": "GO:0005730"
}